{
  "gene_symbol": "FBXO22",
  "gene_name": "F-box only protein 22",
  "gene": "UniProtKB:Q8NEZ5",
  "term_label": "positive regulation of proteasomal ubiquitin-dependent protein catabolic process",
  "term_id": "GO:0032436"
}